{
  "term_id": "GO:0002098",
  "gene_name": "Protein KTI12 homolog",
  "term_label": "tRNA wobble uridine modification",
  "gene": "UniProtKB:Q96EK9",
  "gene_symbol": "KTI12"
}